vacuolar transporter chaperone complex [GO:0033254] (cellular component) References: PMID:11823419, PMID:17079729, PMID:34544285 Relationships: is a type of membrane protein complex [GO:0098796]; is a type of intracellular protein-containing complex [GO:0140535] Definition: A protein complex that contains four related proteins that have been implicated in several membrane-related processes, such as sorting of H+-translocating ATPases, endocytosis, ER-Golgi trafficking, vacuole fusion, vacuolar polyphosphate homeostasis and the microautophagic scission of vesicles into the vacuolar lumen. The complex is enriched at the vacuolar membrane, but also found in other cellular compartments, including the ER and the cell periphery. In Saccharomyces, the subunits are Vtc1p, Vtc2p, Vtc3p and Vtc4p. Also known as: VTC complex